regulation of plasma membrane bounded cell projection organization [GO:0120035] (biological process) Definition: Any process that modulates the frequency, rate or extent of a process involved in the formation, arrangement of constituent parts, or disassembly of plasma membrane bounded cell projections. Subtypes: GO:0007027, regulation of neuron projection development [GO:0010975], regulation of microvillus organization [GO:0032530], regulation of plasma membrane bounded cell projection assembly [GO:0120032], regulation of lamellipodium organization [GO:1902743], GO:1902950 Sources: GOC:krc Relationships: is a type of regulation of cell projection organization [GO:0031344]; regulates plasma membrane bounded cell projection organization [GO:0120036]